host cell mitochondrial envelope [GO:0044190] (cellular component) Relationships: is_a GO:0033655; is part of GO:0033650 Sources: GOC:jl Definition: The double lipid bilayer enclosing the host cell mitochondrion and separating its contents from the host cell cytoplasm; includes the intermembrane space.